{
  "gene_name": "Collagen alpha-2(XI) chain",
  "gene_symbol": "COL11A2",
  "term_id": "GO:0030020",
  "term_label": "extracellular matrix structural constituent conferring tensile strength",
  "gene": "UniProtKB:P13942"
}